{
  "term_label": "signal transduction",
  "term_id": "GO:0007165",
  "gene": "UniProtKB:Q68BL7",
  "gene_symbol": "OLFML2A",
  "gene_name": "Olfactomedin-like protein 2A"
}